{
  "term_id": "UNKNOWN:0001",
  "gene_name": "Retinoschisin",
  "term_label": "Unknown molecular function",
  "gene_symbol": "RS1",
  "gene": "UniProtKB:O15537"
}